right middle basal body pair [GO:0097565] (cellular component) Note: Due to the asymmetric nature of the Giardia trophozoite, this term is defined spatially as the trophozoite is viewed from the dorsal side, with the two nuclei dorsal to the ventral disc, and the ventral disc toward the anterior. References: PMID:16607022, PMID:5961344 Sources: GOC:giardia, ISBN:9780124260207 Definition: Set of two basal bodies found in Giardia species (trophozoite stage). It comprises the caudal and posteriolateral basal bodies located to the left of the right nucleus of the trophozoite when viewed dorsally. Relationships: is a type of GO:0110165; is part of GO:0042995; has part right posteriolateral basal body [GO:1902674]; BFO_0000051 GO:1902678